retinal dehydrogenase (NAD+) activity [GO:0001758] (molecular function) Relationships: is a type of aldehyde dehydrogenase (NAD+) activity [GO:0004029] Definition: Catalysis of the reaction: retinal + NAD+ + H2O = retinoate + NADH. Acts on both 11-trans and 13-cis forms of retinal. Also known as: retinal dehydrogenase activity, cytosolic retinal dehydrogenase activity, retinal:NAD+ oxidoreductase activity Sources: EC:1.2.1.36